regulation of protein metabolic process [GO:0051246] (biological process) Definition: Any process that modulates the frequency, rate or extent of the chemical reactions and pathways involving a protein. Sources: GOC:ai Also known as: regulation of protein metabolism, regulation of cellular protein metabolic process, regulation of cellular protein metabolism Relationships: is a type of GO:0060255; is a type of regulation of primary metabolic process [GO:0080090]; regulates GO:0019538 Subtypes: GO:0006417, regulation of proteolysis [GO:0030162], regulation of protein modification process [GO:0031399], regulation of granulocyte macrophage colony-stimulating factor production [GO:0032645], regulation of hepatocyte growth factor production [GO:0032646], regulation of lymphotoxin A production [GO:0032681], regulation of protein catabolic process [GO:0042176], regulation of hemoglobin biosynthetic process [GO:0046984], GO:0050746, GO:0051247, GO:0051248, regulation of angiotensin metabolic process [GO:0060177], regulation of amyloid precursor protein catabolic process [GO:1902991], regulation of glycoprotein metabolic process [GO:1903018], regulation of protein maturation [GO:1903317], regulation of amyloid fibril formation [GO:1905906]